positive regulation of steroid hormone biosynthetic process [GO:0090031] (biological process) Sources: GOC:dph, GOC:tb Definition: Any process that increases the frequency, rate or extent of the chemical reactions and pathways resulting in the formation of steroid hormones,compounds with a 1, 2, cyclopentanoperhydrophenanthrene nucleus that act as hormones. Subtypes: positive regulation of glucocorticoid biosynthetic process [GO:0031948], positive regulation of aldosterone biosynthetic process [GO:0032349], GO:0045998 Relationships: is a type of positive regulation of steroid biosynthetic process [GO:0010893]; is a type of positive regulation of hormone biosynthetic process [GO:0046886]; is_a regulation of steroid hormone biosynthetic process [GO:0090030]